{
  "term_id": "GO:0006357",
  "gene": "UniProtKB:Q9NR11",
  "gene_name": "Zinc finger protein 302",
  "term_label": "regulation of transcription by RNA polymerase II",
  "gene_symbol": "ZNF302"
}